{
  "term_id": "UNKNOWN:0001",
  "gene": "UniProtKB:Q9ULK4",
  "gene_name": "Mediator of RNA polymerase II transcription subunit 23",
  "term_label": "Unknown molecular function",
  "gene_symbol": "MED23"
}